pancreatic polypeptide receptor activity [GO:0001602] (MF) Definition: Combining with pancreatic polypeptide PP to initiate a change in cell activity. Relationships: is a type of neuropeptide Y receptor activity [GO:0004983] References: PMID:9315606